{
  "gene_name": "Kallistatin",
  "term_label": "Unknown biological process",
  "gene": "UniProtKB:P29622",
  "term_id": "UNKNOWN:0002",
  "gene_symbol": "SERPINA4"
}